{
  "term_id": "UNKNOWN:0003",
  "gene_name": "Protein FAM110B",
  "term_label": "Unknown cellular component",
  "gene_symbol": "FAM110B",
  "gene": "UniProtKB:Q8TC76"
}